precorrin-2 dehydrogenase activity [GO:0043115] (molecular function) Definition: Catalysis of the reaction: NAD+ + precorrin-2 = 2 H+ + NADH + sirohydrochlorin. Relationships: is a type of oxidoreductase activity, acting on the CH-CH group of donors, NAD or NADP as acceptor [GO:0016628] Sources: EC:1.3.1.76, RHEA:15613 Also known as: siroheme synthase activity, 1,3-dimethyluroporphyrinogen III dehydrogenase activity, dihydrosirohydrochlorin dehydrogenase activity, CysG, Met8p, SirC, precorrin-2 oxidase activity, precorrin-2:NAD+ oxidoreductase activity